{
  "gene_symbol": "FBXL3",
  "gene_name": "F-box_LRR-repeat protein 3",
  "term_id": "GO:0031146",
  "gene": "UniProtKB:Q9UKT7",
  "term_label": "SCF-dependent proteasomal ubiquitin-dependent protein catabolic process"
}